{
  "gene_name": "Zinc finger protein 569",
  "gene": "UniProtKB:Q5MCW4",
  "gene_symbol": "ZNF569",
  "term_label": "regulation of transcription by RNA polymerase II",
  "term_id": "GO:0006357"
}